C-C chemokine receptor CCR2 signaling pathway [GO:0038150] (biological process) Definition: The series of molecular signals initiated by a the C-C chemokine type 2 receptor (CCR2) on the surface of a cell binding to one of it's physiological ligands, and ending with the regulation of a downstream cellular process, e.g. transcription. Sources: GOC:nhn, GOC:signaling Relationships: is a type of chemokine-mediated signaling pathway [GO:0070098] Also known as: C-C chemokine receptor type 2 signaling pathway Subtypes: CCL2-activated CCR2 signaling pathway [GO:0038151]